{
  "term_id": "GO:0030425",
  "gene": "UniProtKB:Q8IZD0",
  "gene_symbol": "SAMD14",
  "term_label": "dendrite",
  "gene_name": "Sterile alpha motif domain-containing protein 14"
}